{
  "gene_name": "Myocyte-specific enhancer factor 2D",
  "term_id": "GO:0030154",
  "gene": "UniProtKB:Q14814",
  "gene_symbol": "MEF2D",
  "term_label": "cell differentiation"
}